delta9-tetrahydrocannabinolate synthase activity [GO:0102778] (molecular function) Sources: GOC:pz, RHEA:34135 Definition: Catalysis of the reaction: cannabigerolate + O2 = delta(9)-tetrahydrocannabinolic acid + hydrogen peroxide. Relationships: is a type of GO:0046993